glial cell projection elongation [GO:0106091] (BP) Definition: The process of creating an elongation or projection from a glial cell. References: PMID:27131624 Sources: GOC:ha Relationships: is_a GO:0048858; is part of glial cell development [GO:0021782] Subtypes: glial cell projection elongation involved in axon ensheathment [GO:0106092]